guard cell development [GO:0010441] (biological process) Sources: GOC:tb Relationships: is a type of cell development [GO:0048468]; is part of guard cell differentiation [GO:0010052] Definition: The process whose specific outcome is the progression of the guard cell over time, from its formation to the mature structure.